{
  "gene_symbol": "LRRC4C",
  "term_id": "GO:0050770",
  "gene_name": "Leucine-rich repeat-containing protein 4C",
  "term_label": "regulation of axonogenesis",
  "gene": "UniProtKB:Q9HCJ2"
}